{
  "gene_name": "Protein FAM13A",
  "term_label": "Unknown cellular component",
  "gene": "UniProtKB:O94988",
  "gene_symbol": "FAM13A",
  "term_id": "UNKNOWN:0003"
}